positive regulation of cell killing [GO:0031343] (biological process) Subtypes: positive regulation of leukocyte mediated cytotoxicity [GO:0001912], GO:0051712, GO:1903661 Relationships: is_a regulation of cell killing [GO:0031341]; is a type of positive regulation of cellular process [GO:0048522]; positively regulates cell killing [GO:0001906] Also known as: up regulation of cell killing, up-regulation of cell killing, upregulation of cell killing, activation of cell killing, stimulation of cell killing Definition: Any process that activates or increases the frequency, rate or extent of cell killing. Sources: GOC:mah